{
  "gene": "UniProtKB:P49146",
  "term_id": "GO:0001601",
  "gene_symbol": "NPY2R",
  "term_label": "peptide YY receptor activity",
  "gene_name": "Neuropeptide Y receptor type 2"
}